{
  "gene": "UniProtKB:A0A087WV53",
  "term_label": "Unknown cellular component",
  "term_id": "UNKNOWN:0003",
  "gene_name": "SPEG neighbor protein",
  "gene_symbol": "SPEGNB"
}